{
  "term_label": "Unknown biological process",
  "gene_symbol": "ANKRD55",
  "gene": "UniProtKB:Q3KP44",
  "gene_name": "Ankyrin repeat domain-containing protein 55",
  "term_id": "UNKNOWN:0002"
}